{
  "gene_name": "ATP-binding cassette sub-family C member 10",
  "gene": "UniProtKB:Q5T3U5",
  "gene_symbol": "ABCC10",
  "term_id": "GO:0005886",
  "term_label": "plasma membrane"
}